{
  "gene_symbol": "CCNJL",
  "gene_name": "Cyclin-J-like protein",
  "gene": "UniProtKB:Q8IV13",
  "term_id": "GO:0000307",
  "term_label": "cyclin-dependent protein kinase holoenzyme complex"
}